{
  "gene": "UniProtKB:D6RIA3",
  "term_label": "Unknown molecular function",
  "gene_name": "Uncharacterized protein C4orf54",
  "term_id": "UNKNOWN:0001",
  "gene_symbol": "C4orf54"
}